{
  "term_id": "GO:0080132",
  "gene_name": "Fatty acid 2-hydroxylase",
  "gene_symbol": "FA2H",
  "gene": "UniProtKB:Q7L5A8",
  "term_label": "fatty acid 2-hydroxylase activity"
}